{
  "term_label": "multivesicular body",
  "gene_symbol": "CHMP4C",
  "gene": "UniProtKB:Q96CF2",
  "gene_name": "Charged multivesicular body protein 4c",
  "term_id": "GO:0005771"
}